{
  "gene": "UniProtKB:Q53GS7",
  "gene_name": "mRNA export factor GLE1",
  "gene_symbol": "GLE1",
  "term_id": "GO:0000822",
  "term_label": "inositol hexakisphosphate binding"
}